{
  "gene_symbol": "WNT2B",
  "term_label": "canonical Wnt signaling pathway",
  "gene": "UniProtKB:Q93097",
  "gene_name": "Protein Wnt-2b",
  "term_id": "GO:0060070"
}